Lewy body formation [GO:0140121] (biological process) Definition: The aggregation, arrangement and bonding together of a set of components to form a Lewy body. References: PMID:15158159 Relationships: is a type of inclusion body assembly [GO:0070841] Regulation: regulated by regulation of Lewy body formation [GO:0140122]; negatively regulated by negative regulation of Lewy body formation [GO:0140123]; positively regulated by positive regulation of Lewy body formation [GO:0140124]